{
  "gene": "UniProtKB:Q8TB45",
  "term_label": "negative regulation of TORC1 signaling",
  "gene_symbol": "DEPTOR",
  "gene_name": "DEP domain-containing mTOR-interacting protein",
  "term_id": "GO:1904262"
}